{
  "term_id": "GO:0004364",
  "gene_symbol": "GSTA3",
  "gene": "UniProtKB:Q16772",
  "gene_name": "Glutathione S-transferase A3",
  "term_label": "glutathione transferase activity"
}